{
  "term_id": "UNKNOWN:0002",
  "gene_symbol": "GPS1",
  "gene": "UniProtKB:Q13098",
  "gene_name": "COP9 signalosome complex subunit 1",
  "term_label": "Unknown biological process"
}